{
  "gene_symbol": "STAT5B",
  "term_label": "cytoplasm",
  "gene": "UniProtKB:P51692",
  "gene_name": "Signal transducer and activator of transcription 5B",
  "term_id": "GO:0005737"
}